{
  "gene": "UniProtKB:Q53S08",
  "gene_symbol": "RAB6D",
  "term_id": "GO:1903292",
  "gene_name": "Ras-related protein Rab-6D",
  "term_label": "protein localization to Golgi membrane"
}